vesicle lumen [GO:0031983] (cellular component) Sources: GOC:mah, GOC:vesicles Definition: The volume enclosed by the membrane or protein that forms a vesicle. Relationships: is a type of organelle lumen [GO:0043233]; is part of GO:0031982 Subtypes: GO:0060205, GO:0097489